{
  "gene_name": "ER membrane protein complex subunit 8",
  "gene_symbol": "EMC8",
  "gene": "UniProtKB:O43402",
  "term_label": "EMC complex",
  "term_id": "GO:0072546"
}